{
  "term_label": "SCF-dependent proteasomal ubiquitin-dependent protein catabolic process",
  "gene_symbol": "FBXL8",
  "term_id": "GO:0031146",
  "gene": "UniProtKB:Q96CD0",
  "gene_name": "F-box_LRR-repeat protein 8"
}